{
  "gene_name": "SRSF protein kinase 1",
  "term_label": "cytoplasm",
  "gene": "UniProtKB:Q96SB4",
  "term_id": "GO:0005737",
  "gene_symbol": "SRPK1"
}